{
  "term_id": "GO:0005634",
  "gene_name": "SMC5-SMC6 complex localization factor protein 1",
  "gene_symbol": "SLF1",
  "term_label": "nucleus",
  "gene": "UniProtKB:Q9BQI6"
}